{
  "term_id": "GO:0005886",
  "gene_name": "Signal-regulatory protein gamma",
  "gene": "UniProtKB:Q9P1W8",
  "term_label": "plasma membrane",
  "gene_symbol": "SIRPG"
}